{
  "gene_symbol": "IFT20",
  "term_id": "GO:0043005",
  "gene": "UniProtKB:Q8IY31",
  "term_label": "neuron projection",
  "gene_name": "Intraflagellar transport protein 20 homolog"
}